{
  "gene": "UniProtKB:Q9NRW1",
  "gene_symbol": "RAB6B",
  "gene_name": "Ras-related protein Rab-6B",
  "term_label": "Golgi apparatus",
  "term_id": "GO:0005794"
}